{
  "gene_symbol": "CSF1R",
  "gene": "UniProtKB:P07333",
  "term_id": "GO:0043235",
  "gene_name": "Macrophage colony-stimulating factor 1 receptor",
  "term_label": "receptor complex"
}